response to oxidative stress [GO:0006979] (biological process) Subtypes: response to reactive oxygen species [GO:0000302], response to hydroperoxide [GO:0033194], cellular response to oxidative stress [GO:0034599], GO:0070994, GO:0080183 Relationships: is a type of response to stress [GO:0006950] Definition: Any process that results in a change in state or activity of a cell or an organism (in terms of movement, secretion, enzyme production, gene expression, etc.) as a result of oxidative stress, a state often resulting from exposure to high levels of reactive oxygen species, e.g. superoxide anions, hydrogen peroxide (H2O2), and hydroxyl radicals. References: PMID:12115731 Sources: GOC:jl Regulation: regulated by GO:1902882; negatively regulated by negative regulation of response to oxidative stress [GO:1902883]; positively regulated by positive regulation of response to oxidative stress [GO:1902884]